{
  "gene": "UniProtKB:Q13822",
  "term_id": "GO:0004528",
  "gene_name": "Ectonucleotide pyrophosphatase_phosphodiesterase family member 2",
  "gene_symbol": "ENPP2",
  "term_label": "phosphodiesterase I activity"
}